{
  "gene_name": "HAUS augmin-like complex subunit 8",
  "term_id": "GO:0007098",
  "gene": "UniProtKB:Q9BT25",
  "term_label": "centrosome cycle",
  "gene_symbol": "HAUS8"
}